{
  "gene": "UniProtKB:A0A804HJT0",
  "gene_symbol": "A0A804HJT0",
  "term_id": "UNKNOWN:0003",
  "gene_name": "Uncharacterized protein",
  "term_label": "Unknown cellular component"
}